G protein-coupled GABA receptor activity [GO:0004965] (molecular function) Definition: Combining with the amino acid gamma-aminobutyric acid (GABA, 4-aminobutyrate) and transmitting the signal across the membrane by activating an associated G-protein; promotes the exchange of GDP for GTP on the alpha subunit of a heterotrimeric G-protein complex. Also known as: G-protein coupled GABA receptor activity, GABA-B receptor activity, metabotropic GABA receptor Sources: GOC:ai, GOC:bf, IUPHAR_RECEPTOR:1276, Wikipedia:GABAB_receptor Relationships: is a type of G protein-coupled receptor activity [GO:0004930]; is a type of GABA receptor activity [GO:0016917]